{
  "term_label": "positive regulation of NLRP3 inflammasome complex assembly",
  "gene_symbol": "NEK7",
  "term_id": "GO:1900227",
  "gene_name": "Serine_threonine-protein kinase Nek7",
  "gene": "UniProtKB:Q8TDX7"
}